{
  "gene_symbol": "NFASC",
  "term_id": "GO:0007420",
  "gene": "UniProtKB:O94856",
  "term_label": "brain development",
  "gene_name": "Neurofascin"
}